negative regulation of double-strand break repair [GO:2000780] (biological process) Subtypes: negative regulation of double-strand break repair via single-strand annealing [GO:1901291], negative regulation of double-strand break repair via homologous recombination [GO:2000042], negative regulation of double-strand break repair via nonhomologous end joining [GO:2001033] Relationships: is a type of GO:0045738; is_a regulation of double-strand break repair [GO:2000779]; negatively regulates double-strand break repair [GO:0006302] Sources: GOC:BHF Definition: Any process that stops, prevents or reduces the frequency, rate or extent of double-strand break repair.